{
  "term_id": "GO:0000122",
  "gene_symbol": "NFX1",
  "term_label": "negative regulation of transcription by RNA polymerase II",
  "gene_name": "Transcriptional repressor NF-X1",
  "gene": "UniProtKB:Q12986"
}